peptide-lysine-N-succinyltransferase activity [GO:0106076] (molecular function) References: PMID:29211711 Definition: Catalysis of the reaction: succinyl-CoA + lysine in peptide = CoA + N-succinyl-lysine-peptide. Relationships: is a type of GO:0106075